{
  "gene_symbol": "DCLRE1C",
  "term_id": "GO:0035312",
  "gene_name": "Protein artemis",
  "term_label": "5'-3' DNA exonuclease activity",
  "gene": "UniProtKB:Q96SD1"
}